{
  "term_label": "P granule organization",
  "gene_symbol": "TDRD7",
  "gene": "UniProtKB:Q8NHU6",
  "gene_name": "Tudor domain-containing protein 7",
  "term_id": "GO:0030719"
}